{
  "term_id": "GO:0008934",
  "gene": "UniProtKB:P29218",
  "gene_symbol": "IMPA1",
  "term_label": "inositol monophosphate 1-phosphatase activity",
  "gene_name": "Inositol monophosphatase 1"
}